vitamin biosynthetic process [GO:0009110] (BP) Definition: The chemical reactions and pathways resulting in the formation of a vitamin, one of a number of unrelated organic substances that occur in many foods in small amounts and that are necessary in trace amounts for the normal metabolic functioning of the body. Sources: GOC:go_curators, ISBN:0198506732 Also known as: vitamin anabolism, vitamin biosynthesis, vitamin formation, vitamin synthesis Relationships: is a type of vitamin metabolic process [GO:0006766]; is a type of small molecule biosynthetic process [GO:0044283] Subtypes: GO:0042362, water-soluble vitamin biosynthetic process [GO:0042364]